(S)-2-methylmalate dehydratase activity [GO:0047510] (molecular function) Also known as: (+)-citramalate hydro-lyase activity, (+)-citramalic hydro-lyase activity, (S)-2-methylmalate hydro-lyase (2-methylfumarate-forming), (S)-2-methylmalate hydro-lyase activity, L-citramalate hydrolase activity, citramalate dehydratase activity, mesaconase activity, mesaconate hydratase activity, mesaconate mesaconase activity Relationships: is a type of GO:0016836 Definition: Catalysis of the reaction: S-citramalate = H2O + mesaconate. Sources: RHEA:13529